response to doxorubicin [GO:1902520] (biological process) Note: Note that this term is in the subset of terms that should not be used for direct manual annotation of gene products. It was created to be used for cross-referencing by other ontologies. Direct annotations to this term may be amended during annotation QC. References: PMID:23648065 Sources: GOC:TermGenie, GOC:dw Definition: Any process that results in a change in state or activity of a cell or an organism (in terms of movement, secretion, enzyme production, gene expression, etc.) as a result of a doxorubicin stimulus. Relationships: is a type of response to alcohol [GO:0097305]; is a type of response to ketone [GO:1901654]; is a type of response to nitrogen compound [GO:1901698]; is a type of response to glycoside [GO:1903416]